creatinine metabolic process [GO:0046449] (biological process) Subtypes: creatinine catabolic process [GO:0006602] Sources: ISBN:0198506732 Relationships: is_a GO:0072338 Also known as: creatinine metabolism Definition: The chemical reactions and pathways involving creatinine, 2-amino-1,5-dihydro-1-methyl-4H-imidazol-4-one, an end product of creatine metabolism and a normal constituent of urine.